{
  "term_id": "GO:0017134",
  "gene_symbol": "FGFRL1",
  "gene": "UniProtKB:Q8N441",
  "term_label": "fibroblast growth factor binding",
  "gene_name": "Fibroblast growth factor receptor-like 1"
}